{
  "gene_name": "Hydroxymethylglutaryl-CoA synthase, cytoplasmic",
  "gene_symbol": "HMGCS1",
  "term_id": "GO:0006084",
  "gene": "UniProtKB:Q01581",
  "term_label": "acetyl-CoA metabolic process"
}